{
  "term_id": "GO:0010468",
  "gene_name": "Heterogeneous nuclear ribonucleoprotein D-like",
  "gene_symbol": "HNRNPDL",
  "term_label": "regulation of gene expression",
  "gene": "UniProtKB:O14979"
}